{
  "term_label": "positive regulation of MAPK cascade",
  "gene": "UniProtKB:Q9NSA1",
  "gene_symbol": "FGF21",
  "gene_name": "Fibroblast growth factor 21",
  "term_id": "GO:0043410"
}